{
  "term_id": "UNKNOWN:0003",
  "gene_symbol": "ERVK3-1",
  "term_label": "Unknown cellular component",
  "gene": "UniProtKB:B3KNS4",
  "gene_name": "Endogenous retrovirus group K3 member 1"
}